lipoic acid binding [GO:0031405] (molecular function) Relationships: is a type of fatty acid binding [GO:0005504]; is a type of heterocyclic compound binding [GO:1901363]; is a type of sulfur compound binding [GO:1901681] Definition: Binding to lipoic acid, 1,2-dithiolane-3-pentanoic acid. Sources: GOC:mah, ISBN:0198506732